{
  "term_label": "peptide receptor activity",
  "gene": "UniProtKB:P51841",
  "gene_symbol": "GUCY2F",
  "gene_name": "Retinal guanylyl cyclase 2",
  "term_id": "GO:0001653"
}